{
  "term_label": "regulation of DNA-templated transcription",
  "gene": "UniProtKB:Q9NVM4",
  "term_id": "GO:0006355",
  "gene_symbol": "PRMT7",
  "gene_name": "Protein arginine N-methyltransferase 7"
}